{
  "gene_symbol": "GABARAPL1",
  "gene_name": "Gamma-aminobutyric acid receptor-associated protein-like 1",
  "term_label": "autophagosome membrane",
  "term_id": "GO:0000421",
  "gene": "UniProtKB:Q9H0R8"
}